{
  "gene_symbol": "TUFT1",
  "term_id": "GO:0031674",
  "gene": "UniProtKB:Q9NNX1",
  "term_label": "I band",
  "gene_name": "Tuftelin"
}